{
  "gene": "UniProtKB:Q6PI47",
  "gene_symbol": "KCTD18",
  "gene_name": "BTB_POZ domain-containing protein KCTD18",
  "term_label": "Unknown molecular function",
  "term_id": "UNKNOWN:0001"
}